{
  "gene_symbol": "CAVIN3",
  "term_label": "caveola",
  "gene": "UniProtKB:Q969G5",
  "gene_name": "Caveolae-associated protein 3",
  "term_id": "GO:0005901"
}